regulation of DNA strand elongation [GO:0060382] (biological process) Definition: Any process that modulates the rate, frequency or extent of DNA strand elongation. DNA strand elongation is the DNA metabolic process in which an existing DNA strand is extended by activities including the addition of nucleotides to the 3' end of the strand. Relationships: is a type of regulation of DNA metabolic process [GO:0051052]; regulates DNA strand elongation [GO:0022616] Subtypes: GO:0060383 Sources: GOC:mah